{
  "gene": "UniProtKB:P53803",
  "term_id": "GO:0003899",
  "gene_name": "DNA-directed RNA polymerases I, II, and III subunit RPABC4",
  "gene_symbol": "POLR2K",
  "term_label": "DNA-directed RNA polymerase activity"
}